mannosyl-oligosaccharide 1,2-alpha-mannosidase complex [GO:0106055] (cellular component) Note: An example is MNL1 (P38888) in Saccharomyces cerevisiae. PMID:19124653 (by physical interaction evidence). Relationships: is a type of endoplasmic reticulum protein-containing complex [GO:0140534]; is a type of catalytic complex [GO:1902494]; is part of endoplasmic reticulum lumen [GO:0005788] Definition: A protein complex capable of catalysing the hydrolysis of the terminal (1->2)-linked alpha-D-mannose residues in an oligo-mannose oligosaccharide. References: PMID:21700223 Sources: GOC:bhm